{
  "gene_name": "Transmembrane prolyl 4-hydroxylase",
  "term_label": "regulation of erythrocyte differentiation",
  "term_id": "GO:0045646",
  "gene": "UniProtKB:Q9NXG6",
  "gene_symbol": "P4HTM"
}